{
  "gene_name": "Zinc finger protein 878",
  "gene": "UniProtKB:C9JN71",
  "gene_symbol": "ZNF878",
  "term_label": "nucleus",
  "term_id": "GO:0005634"
}